positive regulation of mitochondrial electron transport, NADH to ubiquinone [GO:1902958] (biological process) References: PMID:23530063 Sources: GOC:TermGenie, GOC:dph, GO_REF:0000058 Also known as: positive regulation of oxidative phosphorylation, NADH to ubiquinone, up regulation of mitochondrial electron transport, NADH to ubiquinone, up regulation of oxidative phosphorylation, NADH to ubiquinone, up-regulation of mitochondrial electron transport, NADH to ubiquinone, up-regulation of oxidative phosphorylation, NADH to ubiquinone, upregulation of mitochondrial electron transport, NADH to ubiquinone, upregulation of oxidative phosphorylation, NADH to ubiquinone, activation of mitochondrial electron transport, NADH to ubiquinone, activation of oxidative phosphorylation, NADH to ubiquinone, activation of complex I (NADH to ubiquinone), positive regulation of complex I (NADH to ubiquinone), up regulation of complex I (NADH to ubiquinone), up-regulation of complex I (NADH to ubiquinone), upregulation of complex I (NADH to ubiquinone) Relationships: is a type of positive regulation of cellular respiration [GO:1901857]; is a type of GO:1902956; positively regulates mitochondrial electron transport, NADH to ubiquinone [GO:0006120] Definition: Any process that activates or increases the frequency, rate or extent of mitochondrial electron transport, NADH to ubiquinone.